maintenance of location in cell [GO:0051651] (biological process) Definition: Any process in which a substance or cellular entity, such as a protein complex or organelle, is maintained in a specific location within, or in the membrane of, a cell, and is prevented from moving elsewhere. Relationships: is a type of cellular process [GO:0009987]; is a type of GO:0051235; is part of cellular localization [GO:0051641] Also known as: cellular retention, cellular sequestering, cellular storage, intracellular retention, intracellular sequestering, intracellular storage, maintenance of intracellular localization, maintenance of localization within cell, retention within cell, sequestering within cell, storage within cell, maintenance of cellular localization, maintenance of localization in cell Sources: GOC:ai Subtypes: maintenance of protein location in cell [GO:0032507], vacuolar sequestering [GO:0043181], maintenance of pole plasm mRNA location [GO:0046594], sequestering of calcium ion [GO:0051208], maintenance of organelle location [GO:0051657], maintenance of protein complex location in cytoplasm [GO:0098545]